{
  "gene_symbol": "STX1B",
  "gene_name": "Syntaxin-1B",
  "term_id": "GO:0031201",
  "gene": "UniProtKB:P61266",
  "term_label": "SNARE complex"
}